{
  "term_id": "GO:0007163",
  "term_label": "establishment or maintenance of cell polarity",
  "gene_symbol": "RAC1",
  "gene": "UniProtKB:P63000",
  "gene_name": "Ras-related C3 botulinum toxin substrate 1"
}